{
  "gene_symbol": "WDR20",
  "term_id": "GO:2000059",
  "gene": "UniProtKB:Q8TBZ3",
  "gene_name": "WD repeat-containing protein 20",
  "term_label": "negative regulation of ubiquitin-dependent protein catabolic process"
}